{
  "gene_name": "Transcription factor HES-5",
  "term_id": "GO:0030182",
  "gene": "UniProtKB:Q5TA89",
  "term_label": "neuron differentiation",
  "gene_symbol": "HES5"
}